negative regulation of membrane hyperpolarization [GO:1902631] (biological process) Definition: Any process that stops, prevents or reduces the frequency, rate or extent of membrane hyperpolarization. Also known as: down regulation of membrane hyperpolarization, down-regulation of membrane hyperpolarization, downregulation of membrane hyperpolarization, inhibition of membrane hyperpolarization Relationships: is a type of negative regulation of biological process [GO:0048519]; is a type of regulation of membrane hyperpolarization [GO:1902630]; negatively regulates GO:0060081 References: PMID:23223304 Sources: GOC:TermGenie, GO_REF:0000058